{
  "term_label": "transcription preinitiation complex",
  "gene_symbol": "ERCC3",
  "term_id": "GO:0097550",
  "gene_name": "General transcription and DNA repair factor IIH helicase subunit XPB",
  "gene": "UniProtKB:P19447"
}